{
  "gene": "UniProtKB:O43908",
  "gene_name": "NKG2-F type II integral membrane protein",
  "term_id": "GO:0045954",
  "term_label": "positive regulation of natural killer cell mediated cytotoxicity",
  "gene_symbol": "KLRC4"
}